{
  "gene_symbol": "FAF1",
  "gene": "UniProtKB:Q9UNN5",
  "term_id": "GO:0036503",
  "gene_name": "FAS-associated factor 1",
  "term_label": "ERAD pathway"
}